{
  "gene_name": "Sterol regulatory element-binding protein 1",
  "gene": "UniProtKB:P36956",
  "gene_symbol": "SREBF1",
  "term_id": "GO:0000981",
  "term_label": "DNA-binding transcription factor activity, RNA polymerase II-specific"
}